hyphal growth [GO:0030448] (biological process) Definition: Growth of fungi as threadlike, tubular structures that may contain multiple nuclei and may or may not be divided internally by septa, or cross-walls. Sources: GOC:mcc, ISBN:0471522295 Also known as: formation of symbiont invasive hypha in host, formation of symbiont invasive hypha within host, formation of symbiont invasive hypha within host during symbiotic interaction, invasive hyphal growth, symbiont invasive hypha formation within host Relationships: is a type of GO:0030447